regulation of ureteric bud formation [GO:0072106] (biological process) Definition: Any process that modulates the developmental process pertaining to the initial formation of the ureteric bud from the Wolffian duct. Sources: GOC:mtg_kidney_jan10 Subtypes: positive regulation of ureteric bud formation [GO:0072107] Relationships: is a type of GO:0061217; is a type of regulation of epithelial tube formation [GO:1905276]; is a type of regulation of animal organ morphogenesis [GO:2000027]; regulates ureteric bud formation [GO:0060676]